{
  "gene_symbol": "MYO7A",
  "gene_name": "Unconventional myosin-VIIa",
  "term_id": "GO:0030048",
  "gene": "UniProtKB:Q13402",
  "term_label": "actin filament-based movement"
}